cellular component disassembly involved in execution phase of apoptosis [GO:0006921] (biological process) Also known as: cellular component disassembly involved in apoptotic process, disassembly of cell structures, cellular component disassembly involved in apoptosis Sources: GOC:dph, GOC:mah, GOC:mtg_apoptosis, GOC:tb Definition: The breakdown of structures such as organelles, proteins, or other macromolecular structures during apoptosis. Subtypes: apoptotic nuclear changes [GO:0030262] Relationships: is a type of GO:0022411; is part of execution phase of apoptosis [GO:0097194]